peptidyl-arginine omega-N-methylation [GO:0035247] (biological process) Subtypes: GO:0019918, GO:0019919 References: PMID:14705965 Sources: RESID:AA0067, RESID:AA0068, RESID:AA0069 Relationships: is_a GO:0035246 Definition: The addition of a methyl group onto a terminal nitrogen (omega nitrogen) atom of an arginine residue in a protein.